{
  "term_label": "pyruvate transmembrane transporter activity",
  "gene_symbol": "MPC1L",
  "gene_name": "Mitochondrial pyruvate carrier 1-like protein",
  "term_id": "GO:0050833",
  "gene": "UniProtKB:P0DKB6"
}